{
  "gene": "UniProtKB:A3QJZ6",
  "term_id": "GO:1990756",
  "gene_symbol": "PRAMEF22",
  "term_label": "ubiquitin-like ligase-substrate adaptor activity",
  "gene_name": "PRAME family member 22"
}